positive regulation of apoptotic process involved in morphogenesis [GO:1902339] (biological process) Also known as: up regulation of apoptotic process involved in morphogenesis, up-regulation of apoptotic process involved in morphogenesis, upregulation of apoptotic process involved in morphogenesis, activation of apoptosis involved in morphogenesis, activation of apoptotic process involved in morphogenesis, positive regulation of apoptosis involved in morphogenesis, up regulation of apoptosis involved in morphogenesis, up-regulation of apoptosis involved in morphogenesis, upregulation of apoptosis involved in morphogenesis, activation of apoptosis involved in development, activation of morphogenetic apoptosis, positive regulation of apoptosis involved in development, positive regulation of morphogenetic apoptosis, up regulation of apoptosis involved in development, up regulation of morphogenetic apoptosis, up-regulation of apoptosis involved in development, up-regulation of morphogenetic apoptosis, upregulation of apoptosis involved in development, upregulation of morphogenetic apoptosis Subtypes: positive regulation of apoptotic process involved in mammary gland involution [GO:0060058], positive regulation of mesenchymal cell apoptotic process involved in nephron morphogenesis [GO:0072041], positive regulation of apoptotic process involved in outflow tract morphogenesis [GO:1902258] Definition: Any process that activates or increases the frequency, rate or extent of apoptotic process involved in morphogenesis. Relationships: is a type of regulation of apoptotic process involved in morphogenesis [GO:1902337]; is a type of positive regulation of apoptotic process involved in development [GO:1904747]; positively regulates GO:0060561 References: PMID:12202035 Sources: GOC:TermGenie, GOC:sart